{
  "gene_symbol": "BICD2",
  "term_label": "dynactin binding",
  "gene_name": "Protein bicaudal D homolog 2",
  "gene": "UniProtKB:Q8TD16",
  "term_id": "GO:0034452"
}